olefinic compound metabolic process [GO:0120254] (biological process) Relationships: is a type of metabolic process [GO:0008152] Sources: GOC:krc Definition: The chemical reactions and pathways involving an olefinic compound, any compound which contains a carbon-carbon double bond (aka C=C). Also known as: alkene substituted compound metabolic process, alkene substituted compound metabolism Subtypes: GO:0009687, cinnamic acid ester metabolic process [GO:0009801], cinnamic acid metabolic process [GO:0009803], styrene metabolic process [GO:0018966], GO:0019369, aldosterone metabolic process [GO:0032341], ferulate metabolic process [GO:0033494], cortisol metabolic process [GO:0034650], GO:0036109, progesterone metabolic process [GO:0042448], GO:0042572, retinal metabolic process [GO:0042574], GO:0042854, GO:0043651, GO:0120255, olefinic compound catabolic process [GO:0120256], olefin metabolic process [GO:1900673]